{
  "gene_symbol": "HIP1",
  "gene": "UniProtKB:O00291",
  "term_label": "clathrin adaptor activity",
  "gene_name": "Huntingtin-interacting protein 1",
  "term_id": "GO:0035615"
}